{
  "term_label": "triglyceride catabolic process",
  "term_id": "GO:0019433",
  "gene": "UniProtKB:P41247",
  "gene_name": "Patatin-like phospholipase domain-containing protein 4",
  "gene_symbol": "PNPLA4"
}